histone H3R8 arginine deiminase activity [GO:0140796] (molecular function) Also known as: H3-R8 citrullination, histone H3-R8 arginine deiminase activity, histone-arginine deiminase activity (H3-R8 specific) References: PMID:15339660 Definition: Catalysis of the reaction: H2O + histone H3 L-arginyl (position 8)= histone H3 L-citrullyl (position 8) + NH4+, resulting in histone H3 citrullination at position 8. Relationships: is_a histone H3 arginine deiminase activity [GO:0141057] Note: Comment: Note that the residue position corresponds to the canonical human H3 histone (UniProtKB:P84243); this residue is conserved across all eukaryotes. Residue 1 is the first residue following removal of the initiating Methionine (Met). Note that each histone is encoded by multiple genes, and sequences may vary across different genes within an organism. The substrate for histone deiminase may be methyl-arginine, rather than arginine (see PMID:35197210 and PMID:16567635).